{
  "gene_name": "Prefoldin subunit 5",
  "term_id": "GO:1990115",
  "gene_symbol": "PFDN5",
  "term_label": "RNA polymerase III assembly",
  "gene": "UniProtKB:Q99471"
}